{
  "term_label": "homophilic cell-cell adhesion",
  "gene_name": "Inactive tyrosine-protein kinase 7",
  "term_id": "GO:0007156",
  "gene_symbol": "PTK7",
  "gene": "UniProtKB:Q13308"
}